{
  "gene_name": "Palladin",
  "term_label": "homophilic cell-cell adhesion",
  "gene_symbol": "PALLD",
  "term_id": "GO:0007156",
  "gene": "UniProtKB:Q8WX93"
}